phospholipase binding [GO:0043274] (molecular function) Relationships: is a type of GO:0019899 Definition: Binding to a phospholipase. Sources: GOC:jl